{
  "gene": "UniProtKB:Q96C10",
  "gene_symbol": "DHX58",
  "gene_name": "ATP-dependent RNA helicase DHX58",
  "term_id": "GO:0005737",
  "term_label": "cytoplasm"
}